cellular response to L-phenylalanine derivative [GO:1904387] (biological process) Subtypes: cellular response to thyroxine stimulus [GO:0097069], GO:1904474 Relationships: is a type of cellular response to nitrogen compound [GO:1901699]; is a type of response to L-phenylalanine derivative [GO:1904386] References: PMID:12112407 Sources: GOC:TermGenie, GO_REF:0000071 Definition: Any process that results in a change in state or activity of a cell (in terms of movement, secretion, enzyme production, gene expression, etc.) as a result of a L-phenylalanine derivative stimulus.